{
  "term_id": "GO:0004984",
  "gene_name": "Olfactory receptor 12D2",
  "gene": "UniProtKB:P58182",
  "term_label": "olfactory receptor activity",
  "gene_symbol": "OR12D2"
}